{
  "term_label": "Unknown biological process",
  "term_id": "UNKNOWN:0002",
  "gene_symbol": "PSMD5",
  "gene": "UniProtKB:Q16401",
  "gene_name": "26S proteasome non-ATPase regulatory subunit 5"
}